{
  "term_id": "UNKNOWN:0002",
  "gene": "UniProtKB:Q53GQ0",
  "term_label": "Unknown biological process",
  "gene_symbol": "HSD17B12",
  "gene_name": "Very-long-chain 3-oxoacyl-CoA reductase"
}